{
  "term_label": "alpha-mannosidase activity",
  "term_id": "GO:0004559",
  "gene_name": "Lysosomal alpha-mannosidase",
  "gene_symbol": "MAN2B1",
  "gene": "UniProtKB:O00754"
}